activating MHC class I receptor activity [GO:0032397] (MF) Definition: Combining with a MHC class I protein complex to mediate signaling that activates a lymphocyte. References: PMID:11858820, PMID:9597134 Sources: GOC:add Relationships: is a type of GO:0032393 Subtypes: HLA-A specific activating MHC class I receptor activity [GO:0030108]